{
  "gene": "UniProtKB:Q8NH05",
  "term_label": "olfactory receptor activity",
  "gene_name": "Olfactory receptor 4Q3",
  "term_id": "GO:0004984",
  "gene_symbol": "OR4Q3"
}